{
  "gene_symbol": "DRGX",
  "gene_name": "Dorsal root ganglia homeobox protein",
  "term_label": "regulation of transcription by RNA polymerase II",
  "gene": "UniProtKB:A6NNA5",
  "term_id": "GO:0006357"
}